{
  "gene_symbol": "PKIA",
  "gene": "UniProtKB:P61925",
  "term_id": "GO:0005634",
  "gene_name": "cAMP-dependent protein kinase inhibitor alpha",
  "term_label": "nucleus"
}